otolith mineralization completed early in development [GO:0031173] (biological process) Relationships: is a type of otolith mineralization [GO:0045299] Definition: The formation of otoliths during embryogenesis with completion in early postembryonic development. Formation occurs by precipitation of specific crystal forms of calcium carbonate around an organic core of extracellular matrix proteins. Otoconia (otoliths) are small (~10 micron) dense extracellular particles present in the otolith end organs of the vertebrate inner ear. Also known as: otoconia mineralization, otoconium mineralization References: PMID:15581873 Sources: GOC:dsf